{
  "term_label": "extracellular space",
  "gene": "UniProtKB:Q8WWQ2",
  "gene_name": "Inactive heparanase-2",
  "gene_symbol": "HPSE2",
  "term_id": "GO:0005615"
}